{
  "gene_symbol": "DCLRE1A",
  "gene": "UniProtKB:Q6PJP8",
  "term_id": "GO:0005634",
  "gene_name": "DNA cross-link repair 1A protein",
  "term_label": "nucleus"
}